{
  "gene": "UniProtKB:O95980",
  "term_label": "plasma membrane",
  "gene_name": "Reversion-inducing cysteine-rich protein with Kazal motifs",
  "term_id": "GO:0005886",
  "gene_symbol": "RECK"
}